{
  "term_id": "GO:0030234",
  "gene_symbol": "SCG5",
  "term_label": "enzyme regulator activity",
  "gene_name": "Neuroendocrine protein 7B2",
  "gene": "UniProtKB:P05408"
}